{
  "gene_name": "POC1 centriolar protein homolog B",
  "gene_symbol": "POC1B",
  "gene": "UniProtKB:Q8TC44",
  "term_label": "centriole",
  "term_id": "GO:0005814"
}